{
  "term_label": "RNA binding",
  "gene": "UniProtKB:Q659C4",
  "term_id": "GO:0003723",
  "gene_name": "La-related protein 1B",
  "gene_symbol": "LARP1B"
}